{
  "gene_name": "BTB_POZ domain-containing protein 6",
  "gene": "UniProtKB:Q96KE9",
  "term_id": "GO:0022008",
  "gene_symbol": "BTBD6",
  "term_label": "neurogenesis"
}